{
  "term_id": "GO:0005762",
  "gene": "UniProtKB:Q7Z7H8",
  "gene_symbol": "MRPL10",
  "term_label": "mitochondrial large ribosomal subunit",
  "gene_name": "Large ribosomal subunit protein uL10m"
}